peptide YY receptor activity [GO:0001601] (molecular function) Definition: Combining with gut peptide YY to initiate a change in cell activity. References: PMID:9315606 Relationships: is a type of neuropeptide Y receptor activity [GO:0004983]